{
  "gene_symbol": "VTI1B",
  "gene": "UniProtKB:Q9UEU0",
  "gene_name": "Vesicle transport through interaction with t-SNAREs homolog 1B",
  "term_label": "endoplasmic reticulum membrane",
  "term_id": "GO:0005789"
}